{
  "term_label": "plasma membrane",
  "gene": "UniProtKB:P47775",
  "gene_name": "G-protein coupled receptor 12",
  "gene_symbol": "GPR12",
  "term_id": "GO:0005886"
}